{
  "term_id": "GO:0051015",
  "gene": "UniProtKB:Q9H2D6",
  "term_label": "actin filament binding",
  "gene_name": "TRIO and F-actin-binding protein",
  "gene_symbol": "TRIOBP"
}